snRNA (adenine-N6)-methylation [GO:0120049] (biological process) Relationships: is a type of GO:0040031 References: PMID:28525753 Definition: The posttranscriptional N6-methylation of an adenine residue in an snRNA molecule.